{
  "term_label": "Unknown biological process",
  "term_id": "UNKNOWN:0002",
  "gene_name": "Olfactory receptor 52P1",
  "gene": "UniProtKB:Q8NH57",
  "gene_symbol": "OR52P1"
}